{
  "term_id": "GO:0006357",
  "gene_symbol": "ZNF840P",
  "gene_name": "Putative zinc finger protein 840",
  "gene": "UniProtKB:A6NDX5",
  "term_label": "regulation of transcription by RNA polymerase II"
}